{
  "term_id": "GO:0005737",
  "term_label": "cytoplasm",
  "gene_name": "Volume-regulated anion channel subunit LRRC8A",
  "gene": "UniProtKB:Q8IWT6",
  "gene_symbol": "LRRC8A"
}